{
  "term_label": "plasma membrane",
  "gene_symbol": "PLEK",
  "gene": "UniProtKB:P08567",
  "gene_name": "Pleckstrin",
  "term_id": "GO:0005886"
}